{
  "gene_symbol": "PIP4K2B",
  "gene_name": "Phosphatidylinositol 5-phosphate 4-kinase type-2 beta",
  "gene": "UniProtKB:P78356",
  "term_id": "GO:0046854",
  "term_label": "phosphatidylinositol phosphate biosynthetic process"
}